{
  "gene": "UniProtKB:Q13308",
  "gene_symbol": "PTK7",
  "gene_name": "Inactive tyrosine-protein kinase 7",
  "term_id": "GO:0005911",
  "term_label": "cell-cell junction"
}